{
  "gene": "UniProtKB:Q92600",
  "term_id": "UNKNOWN:0001",
  "gene_name": "CCR4-NOT transcription complex subunit 9",
  "gene_symbol": "CNOT9",
  "term_label": "Unknown molecular function"
}